symbiont-mediated suppression of host signal transduction pathway via antagonism of host cell surface receptor [GO:0141129] (biological process) Also known as: symbiont-mediated perturbation of host signal transduction pathway via antagonism of host cell surface receptor References: PMID:10221874, PMID:22714643 Relationships: is_a GO:0052029 Definition: A process by which a symbiont alters or subverts a host cell surface receptor-mediated signal transduction pathway by binding to and inhibiting the receptor of the pathway. The host is defined as the larger of the organisms involved in a symbiotic interaction.